{
  "term_id": "GO:0001228",
  "gene": "UniProtKB:Q92481",
  "term_label": "DNA-binding transcription activator activity, RNA polymerase II-specific",
  "gene_symbol": "TFAP2B",
  "gene_name": "Transcription factor AP-2-beta"
}